{
  "term_label": "microtubule organizing center organization",
  "gene_symbol": "SDCCAG8",
  "term_id": "GO:0031023",
  "gene_name": "Serologically defined colon cancer antigen 8",
  "gene": "UniProtKB:Q86SQ7"
}